{
  "gene_symbol": "SPARCL1",
  "gene_name": "SPARC-like protein 1",
  "gene": "UniProtKB:Q14515",
  "term_label": "regulation of synapse organization",
  "term_id": "GO:0050807"
}